plastid membrane [GO:0042170] (cellular component) Sources: GOC:mah Relationships: is a type of GO:0031090; is part of plastid envelope [GO:0009526] Definition: Either of the lipid bilayers that surround a plastid and form the plastid envelope. Subtypes: GO:0009527, plastid inner membrane [GO:0009528], chloroplast membrane [GO:0031969], amyloplast membrane [GO:0033097], cyanelle membrane [GO:0033113], etioplast membrane [GO:0034426], chromoplast membrane [GO:0046862], plastid thylakoid membrane [GO:0055035], apicoplast membrane [GO:0160211]